{
  "term_id": "GO:0005737",
  "term_label": "cytoplasm",
  "gene_name": "BTB_POZ domain-containing protein KCTD20",
  "gene_symbol": "KCTD20",
  "gene": "UniProtKB:Q7Z5Y7"
}